{
  "gene_symbol": "Q6ZN92",
  "term_id": "GO:0046081",
  "term_label": "dUTP catabolic process",
  "gene": "UniProtKB:Q6ZN92",
  "gene_name": "Putative inactive deoxyuridine 5'-triphosphate nucleotidohydrolase-like protein FLJ16323"
}